{
  "term_id": "UNKNOWN:0003",
  "gene_name": "tRNA wybutosine-synthesizing protein 5",
  "term_label": "Unknown cellular component",
  "gene_symbol": "TYW5",
  "gene": "UniProtKB:A2RUC4"
}